{
  "gene_name": "T cell receptor beta joining 2-2P (non-functional) (Fragment)",
  "gene": "UniProtKB:A0A0A0MTA2",
  "term_id": "UNKNOWN:0001",
  "term_label": "Unknown molecular function",
  "gene_symbol": "TRBJ2-2P"
}